regulation of peptidoglycan recognition protein signaling pathway [GO:0061058] (biological process) Also known as: regulation of peptidoglycan recognition protein signalling pathway Relationships: is a type of regulation of pattern recognition receptor signaling pathway [GO:0062207]; regulates peptidoglycan recognition protein signaling pathway [GO:0061057] Sources: GOC:dph Subtypes: positive regulation of peptidoglycan recognition protein signaling pathway [GO:0061059], GO:0061060 Definition: Any process that modulates the rate, frequency, or extent of the peptidoglycan recognition protein signaling pathway.